actin filament-based movement [GO:0030048] (biological process) Definition: Movement of organelles or other particles along actin filaments, or sliding of actin filaments past each other, mediated by motor proteins. Subtypes: vesicle transport along actin filament [GO:0030050], nuclear migration along microfilament [GO:0031022], mitochondrion migration along actin filament [GO:0034642], actin-mediated cell contraction [GO:0070252] Regulation: regulated by GO:1903115; positively regulated by positive regulation of actin filament-based movement [GO:1903116] Relationships: is a type of actin filament-based process [GO:0030029] Sources: GOC:BHF, GOC:mah